{
  "gene_symbol": "MTMR6",
  "term_label": "phosphatidylinositol-3,5-bisphosphate phosphatase activity",
  "gene_name": "Myotubularin-related protein 6",
  "term_id": "GO:0106018",
  "gene": "UniProtKB:Q9Y217"
}